{
  "gene": "UniProtKB:F5H4A9",
  "term_label": "Unknown molecular function",
  "term_id": "UNKNOWN:0001",
  "gene_name": "Uncharacterized membrane protein C3orf80",
  "gene_symbol": "C3orf80"
}